{
  "gene_symbol": "PWWP2A",
  "gene": "UniProtKB:Q96N64",
  "term_label": "nucleus",
  "gene_name": "PWWP domain-containing protein 2A",
  "term_id": "GO:0005634"
}